{
  "term_label": "photoreceptor inner segment",
  "gene_name": "Myosin-IIIa",
  "gene_symbol": "MYO3A",
  "gene": "UniProtKB:Q8NEV4",
  "term_id": "GO:0001917"
}